{
  "term_id": "GO:0042357",
  "gene_name": "Thiamine-triphosphatase",
  "gene": "UniProtKB:Q9BU02",
  "gene_symbol": "THTPA",
  "term_label": "thiamine diphosphate metabolic process"
}